{
  "term_id": "GO:0005739",
  "gene": "UniProtKB:P29803",
  "gene_name": "Pyruvate dehydrogenase E1 component subunit alpha, testis-specific form, mitochondrial",
  "gene_symbol": "PDHA2",
  "term_label": "mitochondrion"
}